{
  "gene_symbol": "RNF227",
  "gene_name": "RING finger protein 227",
  "gene": "UniProtKB:A6NIN4",
  "term_label": "ubiquitin protein ligase activity",
  "term_id": "GO:0061630"
}